peptide antigen assembly with MHC class Ib protein complex [GO:0002492] (biological process) References: PMID:15928678 Sources: GOC:add Definition: The binding of a peptide antigen to the antigen binding groove of an MHC class Ib protein complex. Class Ib here refers to non-classical class I molecules, such as those of the HLA-E gene family. Relationships: is a type of peptide antigen assembly with MHC protein complex [GO:0002501]; is part of MHC class Ib protein complex assembly [GO:0002398]; is part of antigen processing and presentation of peptide antigen via MHC class Ib [GO:0002428]